{
  "gene_name": "Chromatin complexes subunit BAP18",
  "term_label": "MLL1 complex",
  "term_id": "GO:0071339",
  "gene_symbol": "BAP18",
  "gene": "UniProtKB:Q8IXM2"
}